regulation of photoperiodism, flowering [GO:2000028] (biological process) Also known as: regulation of photoperiodic control of flowering time, regulation of photoperiodic control of inflorescence development, regulation of response to day length, flowering, regulation of response to night length, flowering, regulation of response to photoperiod, flowering Subtypes: regulation of long-day photoperiodism, flowering [GO:0048586], regulation of short-day photoperiodism, flowering [GO:0048587] Relationships: is_a GO:0048583; regulates GO:0048573 Definition: Any process that modulates the frequency, rate or extent of photoperiodism, flowering. Sources: GOC:obol